{
  "gene_name": "Cyclic nucleotide-gated cation channel alpha-3",
  "gene_symbol": "CNGA3",
  "gene": "UniProtKB:Q16281",
  "term_id": "GO:0030553",
  "term_label": "cGMP binding"
}